{
  "term_id": "GO:0030510",
  "gene": "UniProtKB:Q12841",
  "term_label": "regulation of BMP signaling pathway",
  "gene_name": "Follistatin-related protein 1",
  "gene_symbol": "FSTL1"
}